polyprenyl diphosphate phosphatase activity [GO:0120556] (molecular function) Definition: Catalysis of the dephosphorylation of polyprenyl diphosphates. Relationships: is a type of isoprenoid diphosphate phosphatase activity [GO:0106405] Subtypes: dolichyldiphosphatase activity [GO:0047874], undecaprenyl-diphosphatase activity [GO:0050380], farnesyl diphosphatase activity [GO:0120557] Sources: GOC:curators